positive regulation of macrophage activation [GO:0043032] (biological process) Subtypes: GO:1903980 Relationships: is a type of positive regulation of leukocyte activation [GO:0002696]; is_a regulation of macrophage activation [GO:0043030]; positively regulates macrophage activation [GO:0042116] Definition: Any process that stimulates, induces or increases the rate of macrophage activation. Sources: GOC:jl Also known as: positive regulation of macrophage polarization, up regulation of macrophage activation, up-regulation of macrophage activation, upregulation of macrophage activation, activation of macrophage activation, stimulation of macrophage activation